GPI anchor metabolic process [GO:0006505] (biological process) Sources: ISBN:0198506732 Subtypes: GPI anchor biosynthetic process [GO:0006506], mannosyl diphosphorylinositol ceramide metabolic process [GO:0006676] Also known as: GPI/GSI anchor metabolic process, GPI/GSI anchor metabolism, GPI anchor metabolism, glycosylphosphatidylinositol metabolic process, glycosylphosphatidylinositol metabolism Definition: The chemical reactions and pathways involving glycosylphosphatidylinositol anchors, molecular mechanisms for attaching membrane proteins to the lipid bilayer of cell membranes. Structurally they consist of a molecule of phosphatidylinositol to which is linked, via the C-6 hydroxyl of the inositol, a carbohydrate chain. This chain is in turn linked to the protein through an ethanolamine phosphate group, the amino group of which is in amide linkage with the C-terminal carboxyl of the protein chain, the phosphate group being esterified to the C-6 hydroxyl of the terminal mannose of the core carbohydrate chain. Relationships: is a type of glycolipid metabolic process [GO:0006664]; is a type of phosphatidylinositol metabolic process [GO:0046488]